{
  "gene_symbol": "NCBP1",
  "term_label": "mRNA export from nucleus",
  "gene": "UniProtKB:Q09161",
  "gene_name": "Nuclear cap-binding protein subunit 1",
  "term_id": "GO:0006406"
}